aldonate transmembrane transport [GO:0042873] (biological process) Also known as: aldonate transport Definition: The process in which aldonate is transported across a lipid bilayer, from one side of a membrane to the other. Relationships: is a type of monocarboxylic acid transport [GO:0015718]; is a type of carboxylic acid transmembrane transport [GO:1905039] Subtypes: phosphoglycerate transmembrane transport [GO:0015713], L-idonate transmembrane transport [GO:0015726], GO:0035429, D-galactonate transmembrane transport [GO:0042875], glycerate transmembrane transport [GO:1901975] Sources: GOC:jl